activation of protein kinase C activity [GO:1990051] (biological process) Definition: Any process that initiates the activity of the inactive enzyme protein kinase C. Also known as: PKC activation, protein kinase C activation Relationships: is_a GO:0032147 References: PMID:3156004